{
  "gene": "UniProtKB:P48146",
  "term_id": "GO:0004930",
  "gene_symbol": "NPBWR2",
  "term_label": "G protein-coupled receptor activity",
  "gene_name": "Neuropeptides B_W receptor type 2"
}